{
  "term_label": "endoplasmic reticulum exit site",
  "gene_symbol": "SEC24D",
  "gene_name": "Protein transport protein Sec24D",
  "term_id": "GO:0070971",
  "gene": "UniProtKB:O94855"
}